{
  "gene_name": "Phosphoserine phosphatase",
  "gene_symbol": "PSPH",
  "term_label": "L-phosphoserine phosphatase activity",
  "gene": "UniProtKB:P78330",
  "term_id": "GO:0036424"
}